{
  "term_label": "Unknown biological process",
  "gene": "UniProtKB:Q6ZRV3",
  "term_id": "UNKNOWN:0002",
  "gene_symbol": "LINC00696",
  "gene_name": "Putative uncharacterized protein encoded by LINC00696"
}